host cell [GO:0043657] (cellular component) Sources: GOC:jl Definition: A cell within a host organism. Includes the host plasma membrane and any external encapsulating structures such as the host cell wall and cell envelope. Relationships: is a type of host cellular component [GO:0018995]